{
  "gene_name": "PRELI domain containing protein 3A",
  "term_id": "GO:0005758",
  "gene_symbol": "PRELID3A",
  "gene": "UniProtKB:Q96N28",
  "term_label": "mitochondrial intermembrane space"
}